{
  "gene_symbol": "HLA-DOA",
  "term_label": "peptide antigen assembly with MHC class II protein complex",
  "gene": "UniProtKB:P06340",
  "gene_name": "HLA class II histocompatibility antigen, DO alpha chain",
  "term_id": "GO:0002503"
}